{
  "gene_name": "Glucose-fructose oxidoreductase domain-containing protein 1",
  "gene": "UniProtKB:Q9NXC2",
  "term_label": "Unknown cellular component",
  "gene_symbol": "GFOD1",
  "term_id": "UNKNOWN:0003"
}